{
  "term_id": "GO:0007129",
  "gene_name": "Protein SIX6OS1",
  "term_label": "homologous chromosome pairing at meiosis",
  "gene_symbol": "SIX6OS1",
  "gene": "UniProtKB:Q8N1H7"
}